{
  "term_id": "UNKNOWN:0002",
  "gene_name": "Proline-rich membrane anchor 1",
  "gene": "UniProtKB:Q86XR5",
  "term_label": "Unknown biological process",
  "gene_symbol": "PRIMA1"
}